{
  "term_id": "GO:0000425",
  "gene": "UniProtKB:Q99570",
  "term_label": "pexophagy",
  "gene_symbol": "PIK3R4",
  "gene_name": "Phosphoinositide 3-kinase regulatory subunit 4"
}